8-hydroxyquercitin 8-O-methyltransferase activity [GO:0030761] (molecular function) Relationships: is a type of S-adenosylmethionine-dependent methyltransferase activity [GO:0008757] Sources: EC:2.1.1.88, RHEA:16593 Definition: Catalysis of the reaction: 3,3',4',5,7,8-hexahydroxyflavone + S-adenosyl-L-methionine(1+) = 3,3',4',5,7-pentahydroxy-8-methoxyflavone + S-adenosyl-L-homocysteine + H+. Also known as: 8-hydroxyquercetin 8-O-methyltransferase activity, S-adenosyl-L-methionine:3,3',4',5,7,8-hexahydroxyflavone 8-O-methyltransferase activity, flavonol 8-O-methyltransferase activity, flavonol 8-methyltransferase activity